ER membrane insertion complex [GO:0072379] (cellular component) Also known as: endoplasmic reticulum membrane insertion complex Definition: A protein complex that is involved in the post-translational delivery of tail-anchored (TA) membrane proteins to the endoplasmic reticulum. TA membrane proteins, also called type II transmembrane proteins, contain a single C-terminal transmembrane region. Some ER membrane insertion complex subunits are conserved between different species such as mammals and budding yeast. Subtypes: BAT3 complex [GO:0071818], TRC complex [GO:0072380], multi-pass translocon complex [GO:0160064] References: PMID:20676083, PMID:20850366 Sources: GOC:mah Relationships: is a type of protein-containing complex [GO:0032991]; is part of GO:0005829